{
  "gene": "UniProtKB:Q9UMQ3",
  "gene_symbol": "BARX2",
  "term_id": "GO:0005634",
  "term_label": "nucleus",
  "gene_name": "Homeobox protein BarH-like 2"
}